{
  "term_label": "membrane",
  "gene": "UniProtKB:Q96FZ5",
  "gene_symbol": "CMTM7",
  "term_id": "GO:0016020",
  "gene_name": "CKLF-like MARVEL transmembrane domain-containing protein 7"
}